cellular response to camptothecin [GO:0072757] (biological process) Also known as: cellular response to CPT Definition: Any process that results in a change in state or activity of a cell (in terms of movement, secretion, enzyme production, gene expression, etc.) as a result of a camptothecin stimulus. Sources: GOC:mah Relationships: is_a GO:0071312; is a type of GO:0097306; is a type of response to camptothecin [GO:1901563]